{
  "term_label": "tRNA (m2G10) methyltransferase complex",
  "gene_symbol": "TRMT112",
  "gene_name": "Multifunctional methyltransferase subunit TRM112-like protein",
  "term_id": "GO:0043528",
  "gene": "UniProtKB:Q9UI30"
}